{
  "term_label": "cyclic-nucleotide phosphodiesterase activity",
  "gene_symbol": "MPPED1",
  "gene": "UniProtKB:O15442",
  "term_id": "GO:0004112",
  "gene_name": "Metallophosphoesterase domain-containing protein 1"
}